{
  "gene_symbol": "SCTR",
  "gene": "UniProtKB:P47872",
  "term_label": "adenylate cyclase-modulating G protein-coupled receptor signaling pathway",
  "gene_name": "Secretin receptor",
  "term_id": "GO:0007188"
}